{
  "gene": "UniProtKB:Q709C8",
  "gene_name": "Intermembrane lipid transfer protein VPS13C",
  "term_id": "UNKNOWN:0001",
  "gene_symbol": "VPS13C",
  "term_label": "Unknown molecular function"
}